{
  "gene_symbol": "TUBA3C",
  "term_id": "GO:0005525",
  "term_label": "GTP binding",
  "gene": "UniProtKB:P0DPH7",
  "gene_name": "Tubulin alpha-3C chain"
}